{
  "term_id": "GO:0017059",
  "gene": "UniProtKB:Q53FV1",
  "gene_symbol": "ORMDL2",
  "gene_name": "ORM1-like protein 2",
  "term_label": "serine palmitoyltransferase complex"
}